{
  "gene": "UniProtKB:O14829",
  "gene_name": "Serine_threonine-protein phosphatase with EF-hands 1",
  "term_id": "GO:0004722",
  "gene_symbol": "PPEF1",
  "term_label": "protein serine/threonine phosphatase activity"
}